{
  "term_id": "GO:0003682",
  "gene_name": "Nucleoplasmin-2",
  "gene": "UniProtKB:Q86SE8",
  "gene_symbol": "NPM2",
  "term_label": "chromatin binding"
}